chaperonin ATPase complex [GO:0016465] (cellular component) Subtypes: GroEL-GroES complex [GO:1990220] Definition: Multisubunit protein complex with 2x7 (Type I, in most cells) or 2x8 (Type II, in Archaea) ATP-binding sites involved in maintaining an unfolded polypeptide structure before folding or to entry into mitochondria and chloroplasts. Relationships: is a type of protein folding chaperone complex [GO:0101031]; is part of GO:0005829 References: PMID:24816391